{
  "term_label": "phosphatidylinositol-4,5-bisphosphate binding",
  "term_id": "GO:0005546",
  "gene_name": "Target of rapamycin complex 2 subunit MAPKAP1",
  "gene": "UniProtKB:Q9BPZ7",
  "gene_symbol": "MAPKAP1"
}